regulation of 'de novo' NAD biosynthetic process from L-tryptophan [GO:1905012] (biological process) Subtypes: GO:1905013, positive regulation of 'de novo' NAD biosynthetic process from L-tryptophan [GO:1905014] Relationships: is a type of GO:0090357; is a type of regulation of purine nucleotide biosynthetic process [GO:1900371]; is a type of regulation of NAD metabolic process [GO:1902688]; regulates 'de novo' NAD+ biosynthetic process from L-tryptophan [GO:0034354] Definition: Any process that modulates the frequency, rate or extent of 'de novo' NAD biosynthetic process from L-tryptophan. Also known as: regulation of 'de novo' NAD biosynthetic process from tryptophan, regulation of de novo NAD biosynthetic process from tryptophan References: PMID:12140278, PMID:19843166 Sources: GOC:PARL, GOC:TermGenie, GOC:bf, GO_REF:0000058